{
  "gene_symbol": "PIGP",
  "gene_name": "Phosphatidylinositol N-acetylglucosaminyltransferase subunit P",
  "term_label": "endoplasmic reticulum",
  "term_id": "GO:0005783",
  "gene": "UniProtKB:P57054"
}